{
  "gene": "UniProtKB:Q96C12",
  "term_id": "GO:0005829",
  "gene_symbol": "ARMC5",
  "term_label": "cytosol",
  "gene_name": "Armadillo repeat-containing protein 5"
}